{
  "term_label": "endoplasmic reticulum-Golgi intermediate compartment",
  "gene_symbol": "TMED2",
  "term_id": "GO:0005793",
  "gene": "UniProtKB:Q15363",
  "gene_name": "Transmembrane emp24 domain-containing protein 2"
}